{
  "term_label": "embryonic morphogenesis",
  "gene": "UniProtKB:P28360",
  "gene_symbol": "MSX1",
  "term_id": "GO:0048598",
  "gene_name": "Homeobox protein MSX-1"
}